{
  "gene": "UniProtKB:P06276",
  "term_label": "acetylcholinesterase activity",
  "term_id": "GO:0003990",
  "gene_symbol": "BCHE",
  "gene_name": "Cholinesterase"
}